{
  "term_label": "plasma membrane",
  "gene_name": "Regulator of G-protein signaling 14",
  "gene_symbol": "RGS14",
  "term_id": "GO:0005886",
  "gene": "UniProtKB:O43566"
}